{
  "gene_name": "Baculoviral IAP repeat-containing protein 3",
  "term_label": "nucleus",
  "term_id": "GO:0005634",
  "gene_symbol": "BIRC3",
  "gene": "UniProtKB:Q13489"
}